{
  "term_label": "protein localization to kinetochore involved in kinetochore assembly",
  "gene_symbol": "KNTC1",
  "gene_name": "Kinetochore-associated protein 1",
  "term_id": "GO:1903394",
  "gene": "UniProtKB:P50748"
}